{
  "gene_symbol": "BAG3",
  "term_label": "cytoplasm",
  "term_id": "GO:0005737",
  "gene": "UniProtKB:O95817",
  "gene_name": "BAG family molecular chaperone regulator 3"
}